positive regulation of dauer entry [GO:1905911] (biological process) Also known as: positive regulation of nematode entry into dormancy, up regulation of dauer entry, up regulation of nematode entry into dormancy, up-regulation of dauer entry, up-regulation of nematode entry into dormancy, upregulation of dauer entry, upregulation of nematode entry into dormancy, activation of dauer entry, activation of nematode entry into dormancy Definition: Any process that activates or increases the frequency, rate or extent of dauer entry. References: PMID:21531333 Sources: GOC:TermGenie, GO_REF:0000058 Relationships: is a type of GO:0051094; is a type of regulation of dauer entry [GO:1905909]; positively regulates dauer entry [GO:0043053]